{
  "term_id": "GO:0036002",
  "term_label": "pre-mRNA binding",
  "gene_symbol": "RBM22",
  "gene_name": "Pre-mRNA-splicing factor RBM22",
  "gene": "UniProtKB:Q9NW64"
}